{
  "gene_symbol": "PCDHGA12",
  "term_id": "GO:0050839",
  "term_label": "cell adhesion molecule binding",
  "gene_name": "Protocadherin gamma-A12",
  "gene": "UniProtKB:O60330"
}